{
  "term_id": "GO:0015485",
  "gene_symbol": "OSBPL2",
  "gene_name": "Oxysterol-binding protein-related protein 2",
  "gene": "UniProtKB:Q9H1P3",
  "term_label": "cholesterol binding"
}